negative regulation of Toll receptor ligand protein activation cascade [GO:0160035] (biological process) Definition: Any process that stops, prevents or reduces the frequency, rate or extent of Toll receptor ligand protein activation cascade. Relationships: is a type of GO:0160033; is a type of negative regulation of protein activation cascade [GO:2000258]; negatively regulates Toll receptor ligand protein activation cascade [GO:0160032] References: PMID:23632253